ERBB4-ERBB4 signaling pathway [GO:0038138] (biological process) Definition: The series of molecular signals initiated by binding of a ligand to the tyrosine kinase receptor ERBB4, followed by ligand-induced homodimerization of ERBB4 and transmission of the signal into the cell by the homodimeric ERBB4 complex. The pathway ends with regulation of a downstream cellular process, e.g. transcription. References: PMID:16460914 Sources: GOC:signaling Also known as: ERBB4 homodimeric signaling pathway, ERBB4-ERBB4 signalling pathway, HER4-HER4 signaling pathway Relationships: is_a GO:0038130